{
  "term_id": "GO:0043025",
  "term_label": "neuronal cell body",
  "gene_name": "Sorbin and SH3 domain-containing protein 2",
  "gene": "UniProtKB:O94875",
  "gene_symbol": "SORBS2"
}